{
  "gene_name": "Phosphatidylinositol polyphosphate 5-phosphatase type IV",
  "gene": "UniProtKB:Q9NRR6",
  "term_id": "GO:0004439",
  "gene_symbol": "INPP5E",
  "term_label": "phosphatidylinositol-4,5-bisphosphate 5-phosphatase activity"
}